{
  "term_label": "sperm axoneme assembly",
  "gene_symbol": "SPEF2",
  "term_id": "GO:0007288",
  "gene": "UniProtKB:Q9C093",
  "gene_name": "Sperm flagellar protein 2"
}